{
  "term_id": "UNKNOWN:0001",
  "term_label": "Unknown molecular function",
  "gene_name": "Retrotransposon Gag-like protein 5",
  "gene": "UniProtKB:Q5HYW3",
  "gene_symbol": "RTL5"
}